{
  "gene": "UniProtKB:P02647",
  "term_id": "GO:1903561",
  "gene_name": "Apolipoprotein A-I",
  "term_label": "extracellular vesicle",
  "gene_symbol": "APOA1"
}